chloride channel inhibitor activity [GO:0019869] (molecular function) Sources: GOC:mah Definition: Binds to and stops, prevents, or reduces the activity of a chloride channel. Relationships: is a type of GO:0008200; is a type of chloride channel regulator activity [GO:0017081]; negatively regulates chloride channel activity [GO:0005254]